{
  "gene_name": "Palmitoyltransferase ZDHHC9",
  "term_id": "GO:0006612",
  "term_label": "protein targeting to membrane",
  "gene": "UniProtKB:Q9Y397",
  "gene_symbol": "ZDHHC9"
}